{
  "term_id": "GO:0072583",
  "gene_name": "AP-2 complex subunit mu",
  "gene": "UniProtKB:Q96CW1",
  "term_label": "clathrin-dependent endocytosis",
  "gene_symbol": "AP2M1"
}